glycoprotein endo-alpha-1,2-mannosidase activity [GO:0004569] (MF) Sources: EC:3.2.1.130 Definition: Catalysis of the hydrolysis of the terminal alpha-glucosyl-(1,3)-mannosyl unit from Glc-Man(9)-(GlcNAc)(2) oligosaccharide component of the glycoprotein produced in the Golgi membrane. Also known as: endo-alpha-mannosidase activity, endomannosidase activity, glucosyl mannosidase activity, glucosylmannosidase activity, glycoprotein glucosylmannohydrolase activity Relationships: is a type of alpha-mannosidase activity [GO:0004559]